positive regulation of translation [GO:0045727] (biological process) Subtypes: positive regulation of translation in response to stress [GO:0032056], positive regulation of translational elongation [GO:0045901], GO:0045903, positive regulation of translational termination [GO:0045905], GO:0045948, positive regulation of translation, ncRNA-mediated [GO:0045975], GO:0046012, positive regulation of mitochondrial translation [GO:0070131], GO:2000767 Definition: Any process that activates or increases the frequency, rate or extent of the chemical reactions and pathways resulting in the formation of proteins by the translation of mRNA or circRNA. Relationships: is a type of regulation of translation [GO:0006417]; is a type of positive regulation of gene expression [GO:0010628]; is a type of GO:0051247; positively regulates translation [GO:0006412] Sources: GOC:dph, GOC:go_curators, GOC:tb Also known as: positive regulation of protein anabolism, positive regulation of protein biosynthesis, positive regulation of protein biosynthetic process, positive regulation of protein formation, positive regulation of protein synthesis, up regulation of protein biosynthetic process, up-regulation of protein biosynthetic process, upregulation of protein biosynthetic process, activation of protein biosynthetic process, stimulation of protein biosynthetic process